{
  "term_label": "Unknown molecular function",
  "gene_name": "Trafficking protein particle complex subunit 2-like protein",
  "gene_symbol": "TRAPPC2L",
  "gene": "UniProtKB:Q9UL33",
  "term_id": "UNKNOWN:0001"
}